{
  "gene_name": "Protein kintoun",
  "gene": "UniProtKB:Q9NVR5",
  "term_id": "GO:0005737",
  "gene_symbol": "DNAAF2",
  "term_label": "cytoplasm"
}